{
  "gene": "UniProtKB:O60224",
  "gene_symbol": "SSX4",
  "term_label": "Unknown biological process",
  "term_id": "UNKNOWN:0002",
  "gene_name": "Protein SSX4"
}